{
  "gene_symbol": "LINC00269",
  "gene_name": "Putative uncharacterized protein encoded by LINC00269",
  "term_label": "Unknown biological process",
  "term_id": "UNKNOWN:0002",
  "gene": "UniProtKB:Q8N2A0"
}